{
  "gene_name": "Transmembrane protein 222",
  "gene_symbol": "TMEM222",
  "term_id": "UNKNOWN:0001",
  "gene": "UniProtKB:Q9H0R3",
  "term_label": "Unknown molecular function"
}